{
  "gene": "UniProtKB:Q8N377",
  "gene_symbol": "Q8N377",
  "gene_name": "Putative uncharacterized protein LOC387726",
  "term_label": "Unknown cellular component",
  "term_id": "UNKNOWN:0003"
}